{
  "gene_name": "Solute carrier family 52, riboflavin transporter, member 3",
  "term_id": "GO:0032218",
  "gene": "UniProtKB:Q9NQ40",
  "gene_symbol": "SLC52A3",
  "term_label": "riboflavin transport"
}